{
  "gene_symbol": "TMOD1",
  "term_label": "actin filament organization",
  "term_id": "GO:0007015",
  "gene": "UniProtKB:P28289",
  "gene_name": "Tropomodulin-1"
}